{
  "gene_name": "Myosin regulatory light chain 12B",
  "term_id": "GO:0030016",
  "term_label": "myofibril",
  "gene": "UniProtKB:O14950",
  "gene_symbol": "MYL12B"
}